{
  "term_label": "cell migration",
  "gene_name": "Podocalyxin",
  "gene_symbol": "PODXL",
  "gene": "UniProtKB:O00592",
  "term_id": "GO:0016477"
}